{
  "gene_name": "AF4_FMR2 family member 2",
  "term_id": "GO:0050877",
  "gene": "UniProtKB:P51816",
  "term_label": "nervous system process",
  "gene_symbol": "AFF2"
}